{
  "term_id": "GO:0022617",
  "gene_symbol": "KLK4",
  "gene": "UniProtKB:Q9Y5K2",
  "term_label": "extracellular matrix disassembly",
  "gene_name": "Kallikrein-4"
}